{
  "term_label": "nucleus",
  "gene": "UniProtKB:Q14694",
  "gene_symbol": "USP10",
  "gene_name": "Ubiquitin carboxyl-terminal hydrolase 10",
  "term_id": "GO:0005634"
}